{
  "gene_symbol": "SMPD1",
  "term_id": "GO:0061750",
  "gene_name": "Sphingomyelin phosphodiesterase",
  "term_label": "acid sphingomyelin phosphodiesterase activity",
  "gene": "UniProtKB:P17405"
}